apicolateral plasma membrane [GO:0016327] (cellular component) Definition: The apical end of the lateral plasma membrane of epithelial cells. Sources: GOC:hb Also known as: apical lateral plasma membrane Relationships: is a type of GO:0098590